{
  "gene_symbol": "PSAP",
  "gene_name": "Prosaposin",
  "gene": "UniProtKB:P07602",
  "term_id": "GO:0005764",
  "term_label": "lysosome"
}